xenophagy [GO:0098792] (biological process) Relationships: is a type of macroautophagy [GO:0016236]; is part of GO:0098542 References: PMID:19802565, PMID:20159618, PMID:25497060 Sources: GOC:PARL, GOC:autophagy, GOC:pad Regulation: regulated by regulation of xenophagy [GO:1904415]; negatively regulated by negative regulation of xenophagy [GO:1904416]; positively regulated by positive regulation of xenophagy [GO:1904417] Definition: The selective degradation of intracellular pathogen or some part of an intracellular pathogen (e.g. viral capsid) by macroautophagy.